{
  "term_id": "GO:0008331",
  "gene_name": "Voltage-dependent L-type calcium channel subunit beta-3",
  "gene_symbol": "CACNB3",
  "term_label": "high voltage-gated calcium channel activity",
  "gene": "UniProtKB:P54284"
}